{
  "term_label": "carbonate dehydratase activity",
  "gene": "UniProtKB:Q16790",
  "gene_symbol": "CA9",
  "term_id": "GO:0004089",
  "gene_name": "Carbonic anhydrase 9"
}